low molecular weight kininogen binding [GO:0030986] (molecular function) References: PMID:9520414 Sources: GOC:mah Relationships: is a type of kininogen binding [GO:0030984] Also known as: LK binding, LMW kininogen binding Definition: Binding to a kininogen of low molecular mass.